{
  "gene_symbol": "GLOD5",
  "gene": "UniProtKB:A6NK44",
  "gene_name": "Glyoxalase domain-containing protein 5",
  "term_id": "UNKNOWN:0001",
  "term_label": "Unknown molecular function"
}